cellulose metabolic process [GO:0030243] (biological process) Definition: The chemical reactions and pathways involving cellulose, a linear beta1-4 glucan of molecular mass 50-400 kDa with the pyranose units in the -4C1 conformation. Subtypes: GO:0030244, GO:0030245, GO:0052541 Also known as: cellulose metabolism Relationships: is a type of GO:0051273 Sources: GOC:mah, ISBN:0198506732